{
  "term_label": "box H/ACA snoRNP assembly",
  "term_id": "GO:0000493",
  "gene_symbol": "SHQ1",
  "gene": "UniProtKB:Q6PI26",
  "gene_name": "Protein SHQ1 homolog"
}